{
  "term_label": "regulation of transcription by RNA polymerase II",
  "gene_name": "Putative zinc finger protein 137",
  "term_id": "GO:0006357",
  "gene_symbol": "ZNF137P",
  "gene": "UniProtKB:P52743"
}